spontaneous exocytosis of neurotransmitter [GO:0048792] (biological process) Also known as: spontaneous synaptic vesicle exocytosis Sources: GOC:curators Relationships: is a type of neurotransmitter secretion [GO:0007269]; is a type of synaptic vesicle exocytosis [GO:0016079] Definition: The release of a neurotransmitter into the synaptic cleft, where the release step is independent of the presence of calcium ions (Ca2+). The neurotransmitter is contained within a membrane-bounded vesicle, and is released by fusion of the vesicle with the presynaptic plasma membrane of a nerve cell.